negative regulation of cell differentiation involved in phenotypic switching [GO:1905916] (biological process) Relationships: is a type of negative regulation of cell differentiation [GO:0045596]; is a type of GO:1900240; is a type of regulation of cell differentiation involved in phenotypic switching [GO:1905915]; negatively regulates cell differentiation involved in phenotypic switching [GO:0090679] Definition: Any process that stops, prevents or reduces the frequency, rate or extent of cell differentiation involved in phenotypic switching. Also known as: down regulation of cell differentiation involved in phenotypic switching, down-regulation of cell differentiation involved in phenotypic switching, downregulation of cell differentiation involved in phenotypic switching, inhibition of cell differentiation involved in phenotypic switching Subtypes: negative regulation of vascular associated smooth muscle cell differentiation involved in phenotypic switching [GO:1905931] References: PMID:25089138 Sources: GOC:BHF, GOC:BHF_miRNA, GOC:TermGenie, GOC:rph, GO_REF:0000058